regulation of postsynapse assembly [GO:0150052] (BP) References: PMID:16394100, PMID:16672654, PMID:28185854 Sources: GOC:aruk, GOC:bc Relationships: is a type of regulation of synapse assembly [GO:0051963]; is a type of regulation of postsynapse organization [GO:0099175]; regulates postsynapse assembly [GO:0099068] Definition: Any process that modulates the frequency, rate or extent of postsynapse assembly, the aggregation, arrangement and bonding together of a set of components to form a postsynapse.